teichoic acid metabolic process [GO:0046374] (biological process) Definition: The chemical reactions and pathways involving teichoic acid, any polymer occurring in the cell wall, membrane or capsule of Gram-positive bacteria and containing chains of glycerol phosphate or ribitol phosphate residues. Relationships: is a type of macromolecule metabolic process [GO:0043170]; is a type of carbohydrate derivative metabolic process [GO:1901135] Subtypes: teichoic acid biosynthetic process [GO:0019350], teichoic acid catabolic process [GO:0070393] Also known as: teichoic acid metabolism Sources: ISBN:0198506732